regulation of amino acid uptake involved in synaptic transmission [GO:0051941] (BP) Relationships: is a type of regulation of neurotransmitter uptake [GO:0051580]; is a type of regulation of amino acid transport [GO:0051955]; RO_0002211 amino acid neurotransmitter reuptake [GO:0051933] Definition: Any process that modulates the frequency, rate or extent of the directed movement of amino acid neurotransmitters into a neuron or glial cell. Also known as: regulation of amino acid neurotransmitter reuptake, regulation of amino acid neurotransmitter uptake, regulation of amino acid uptake during transmission of nerve impulse Subtypes: GO:0051942, positive regulation of amino acid uptake involved in synaptic transmission [GO:0051943], GO:0051946, regulation of gamma-aminobutyric acid uptake involved in transmission of nerve impulse [GO:0051947] Sources: GOC:ai